{
  "gene_symbol": "CHD5",
  "gene_name": "Chromodomain-helicase-DNA-binding protein 5",
  "term_id": "GO:0140658",
  "gene": "UniProtKB:Q8TDI0",
  "term_label": "ATP-dependent chromatin remodeler activity"
}